{
  "term_label": "nuclear lamina",
  "gene_symbol": "LMNA",
  "gene_name": "Prelamin-A_C",
  "term_id": "GO:0005652",
  "gene": "UniProtKB:P02545"
}